{
  "term_label": "Unknown molecular function",
  "gene_name": "Putative transmembrane protein 183BP",
  "term_id": "UNKNOWN:0001",
  "gene": "UniProtKB:Q1AE95",
  "gene_symbol": "TMEM183BP"
}